{
  "term_id": "GO:0043123",
  "gene": "UniProtKB:Q12802",
  "gene_name": "A-kinase anchor protein 13",
  "term_label": "positive regulation of canonical NF-kappaB signal transduction",
  "gene_symbol": "AKAP13"
}